{
  "gene_symbol": "DNMT3L",
  "gene_name": "DNA (cytosine-5)-methyltransferase 3-like",
  "term_id": "GO:0045892",
  "term_label": "negative regulation of DNA-templated transcription",
  "gene": "UniProtKB:Q9UJW3"
}